negative regulation of cardiac muscle fiber development [GO:0055019] (biological process) Relationships: is a type of negative regulation of cell development [GO:0010721]; is a type of GO:0051154; is a type of regulation of cardiac muscle fiber development [GO:0055018]; negatively regulates cardiac muscle cell development [GO:0055013] Also known as: down regulation of cardiac muscle fiber development, down-regulation of cardiac muscle fiber development, downregulation of cardiac muscle fiber development, negative regulation of cardiac muscle fibre development, inhibition of cardiac muscle fiber development, negative regulation of heart muscle fiber development Sources: GOC:vk Definition: Any process that stops, prevents, or reduces the frequency, rate or extent of cardiac muscle fiber development.